long-chain fatty acid--protein ligase activity [GO:0047474] (molecular function) Sources: EC:6.2.1.19, MetaCyc:6.2.1.19-RXN Also known as: long-chain fatty acid luciferin component ligase activity, long-chain-fatty-acid luciferin component ligase activity, long-chain-fatty-acid-luciferin-component ligase activity, acyl-protein synthetase activity, long-chain-fatty-acid:protein ligase (AMP-forming) Definition: Catalysis of the reaction: a long-chain fatty acid + ATP + L-cysteinyl-[protein] = AMP + diphosphate + S-(long-chain fatty acyl)-L-cysteinyl-[protein]. A long-chain fatty acid has an aliphatic tail containing 13 to 22 carbons. Relationships: is a type of fatty acid ligase activity [GO:0015645] Note: While there is not universal consensus on the lengths of short-, medium-, long- and very-long-chain fatty acids, the GO uses the definitions in ChEBI (see CHEBI:26666, CHEBI:59554, CHEBI:15904 and CHEBI:27283).